{
  "gene_name": "Importin subunit beta-1",
  "term_id": "GO:0008139",
  "gene_symbol": "KPNB1",
  "term_label": "nuclear localization sequence binding",
  "gene": "UniProtKB:Q14974"
}